{
  "term_id": "UNKNOWN:0003",
  "gene_name": "Reprimo-like protein",
  "gene_symbol": "RPRML",
  "gene": "UniProtKB:Q8N4K4",
  "term_label": "Unknown cellular component"
}